{
  "gene": "UniProtKB:P20338",
  "gene_symbol": "RAB4A",
  "term_id": "GO:0003924",
  "gene_name": "Ras-related protein Rab-4A",
  "term_label": "GTPase activity"
}